{
  "term_label": "SNARE complex",
  "gene_symbol": "STX4",
  "gene_name": "Syntaxin-4",
  "gene": "UniProtKB:Q12846",
  "term_id": "GO:0031201"
}